coenzyme F420 binding [GO:0070967] (molecular function) Definition: Binding to F420, the coenzyme or the prosthetic group of various flavoprotein oxidoreductase enzymes. Sources: GOC:dh Relationships: is a type of carboxylic acid binding [GO:0031406]; is a type of carbohydrate derivative binding [GO:0097367]; is a type of heterocyclic compound binding [GO:1901363]